{
  "gene_name": "Pleckstrin homology domain-containing family A member 4",
  "gene_symbol": "PLEKHA4",
  "term_label": "phosphatidylinositol-3,5-bisphosphate binding",
  "term_id": "GO:0080025",
  "gene": "UniProtKB:Q9H4M7"
}